{
  "term_label": "Unknown molecular function",
  "gene_symbol": "POU2AF3",
  "gene": "UniProtKB:A8K830",
  "gene_name": "POU class 2 homeobox associating factor 3",
  "term_id": "UNKNOWN:0001"
}